{
  "gene_name": "Interferon alpha_beta receptor 1",
  "term_label": "plasma membrane",
  "term_id": "GO:0005886",
  "gene": "UniProtKB:P17181",
  "gene_symbol": "IFNAR1"
}